{
  "gene_name": "WASH complex subunit 2C",
  "gene": "UniProtKB:Q9Y4E1",
  "term_id": "GO:0042147",
  "term_label": "retrograde transport, endosome to Golgi",
  "gene_symbol": "WASHC2C"
}